{
  "gene": "UniProtKB:Q9UHP6",
  "term_id": "UNKNOWN:0002",
  "gene_name": "Radial spoke head 14 homolog",
  "gene_symbol": "RSPH14",
  "term_label": "Unknown biological process"
}